regulation of N',N'',N'''-triacetylfusarinine C biosynthetic process [GO:1900695] (biological process) Sources: GOC:TermGenie, GOC:di Definition: Any process that modulates the frequency, rate or extent of N',N'',N'''-triacetylfusarinine C biosynthetic process. Subtypes: negative regulation of N',N'',N'''-triacetylfusarinine C biosynthetic process [GO:1900696], positive regulation of N',N'',N'''-triacetylfusarinine C biosynthetic process [GO:1900697] Relationships: is a type of GO:1900376; regulates N',N'',N'''-triacetylfusarinine C biosynthetic process [GO:1900551] Also known as: regulation of N',N'',N'''-triacetylfusarinine C anabolism, regulation of N',N'',N'''-triacetylfusarinine C biosynthesis, regulation of N',N'',N'''-triacetylfusarinine C formation, regulation of N',N'',N'''-triacetylfusarinine C synthesis